{
  "gene_symbol": "LINC01547",
  "term_label": "Unknown cellular component",
  "gene_name": "Uncharacterized protein encoded by LINC01547",
  "gene": "UniProtKB:P58512",
  "term_id": "UNKNOWN:0003"
}